{
  "term_id": "GO:0005669",
  "term_label": "transcription factor TFIID complex",
  "gene_symbol": "TAF11L6",
  "gene_name": "TATA-box-binding protein-associated factor 11-like protein 6",
  "gene": "UniProtKB:P0DW11"
}